{
  "term_label": "isopentenyl diphosphate biosynthetic process",
  "gene_symbol": "IDI1",
  "term_id": "GO:0009240",
  "gene_name": "Isopentenyl-diphosphate Delta-isomerase 1",
  "gene": "UniProtKB:Q13907"
}